{
  "gene": "UniProtKB:A0A1B0GUT2",
  "gene_name": "Uncharacterized protein C10orf143",
  "gene_symbol": "C10orf143",
  "term_id": "UNKNOWN:0002",
  "term_label": "Unknown biological process"
}